positive regulation of root hair elongation [GO:1902892] (biological process) Definition: Any process that activates or increases the frequency, rate or extent of root hair elongation. References: PMID:22329353 Sources: GOC:TermGenie, GOC:als, GO_REF:0000058 Also known as: up regulation of root hair elongation, up-regulation of root hair elongation, upregulation of root hair elongation, activation of root hair elongation Relationships: is a type of positive regulation of cell growth [GO:0030307]; is a type of GO:0048639; is a type of GO:1902890; is a type of positive regulation of cell maturation [GO:1903431]; positively regulates root hair elongation [GO:0048767]